arachidonate epoxygenase activity [GO:0008392] (molecular function) Definition: Catalysis of an NADPH- and oxygen-dependent reaction that converts arachidonic acid to a cis-epoxyeicosatrienoic acid. References: PMID:10681399, PMID:18952572 Sources: http://lipidlibrary.aocs.org/Lipids/eic_hete/index.htm Also known as: arachidonic acid epoxygenase activity, cytochrome P450 CYP2J5, cytochrome P450 CYP2J6 Relationships: is a type of arachidonate monooxygenase activity [GO:0008391] Subtypes: arachidonate 14,15-epoxygenase activity [GO:0008404], GO:0008405, arachidonate 5,6-epoxygenase activity [GO:0106301], arachidonate 8,9-epoxygenase activity [GO:0106302]